{
  "term_id": "UNKNOWN:0001",
  "term_label": "Unknown molecular function",
  "gene_name": "Spindlin-2B",
  "gene_symbol": "SPIN2B",
  "gene": "UniProtKB:Q9BPZ2"
}